{
  "gene_symbol": "BTN3A1",
  "gene": "UniProtKB:O00481",
  "term_label": "signaling receptor binding",
  "term_id": "GO:0005102",
  "gene_name": "Butyrophilin subfamily 3 member A1"
}